{
  "term_id": "UNKNOWN:0001",
  "gene_name": "Insulin-induced gene 1 protein",
  "gene_symbol": "INSIG1",
  "term_label": "Unknown molecular function",
  "gene": "UniProtKB:O15503"
}